{
  "gene_name": "Protocadherin gamma-A3",
  "term_id": "GO:0007155",
  "gene": "UniProtKB:Q9Y5H0",
  "term_label": "cell adhesion",
  "gene_symbol": "PCDHGA3"
}